{
  "gene_name": "Spermatogenesis-associated protein 6",
  "term_label": "spermatogenesis",
  "gene_symbol": "SPATA6",
  "term_id": "GO:0007283",
  "gene": "UniProtKB:Q9NWH7"
}